{
  "gene": "UniProtKB:Q5QP82",
  "term_label": "Unknown biological process",
  "gene_symbol": "DCAF10",
  "term_id": "UNKNOWN:0002",
  "gene_name": "DDB1- and CUL4-associated factor 10"
}